{
  "term_id": "UNKNOWN:0001",
  "gene_symbol": "TRDJ2",
  "gene": "UniProtKB:A0A075B6V6",
  "gene_name": "T cell receptor delta joining 2 (Fragment)",
  "term_label": "Unknown molecular function"
}